{
  "term_label": "DNA-binding transcription factor activity, RNA polymerase II-specific",
  "term_id": "GO:0000981",
  "gene_name": "Iroquois-class homeodomain protein IRX-2",
  "gene": "UniProtKB:Q9BZI1",
  "gene_symbol": "IRX2"
}